establishment of B cell polarity [GO:0001769] (biological process) Definition: The directed orientation of B cell signaling molecules and associated membrane rafts towards a chemokine gradient of a contact point with an antigen displaying cell. Note: Note that 'antigen displaying cell' in this term encompasses cell types such as follicular dendritic cells which display the unprocessed antigens of a B cell, leading to activation of the B cells and antigen uptake and processing by the B cells. Relationships: is a type of establishment of lymphocyte polarity [GO:0001767]; is part of B cell activation [GO:0042113] Also known as: B cell polarization, B lymphocyte polarization, B-cell polarization, establishment of B lymphocyte polarity, establishment of B-cell polarity, establishment of B-lymphocyte polarity References: PMID:12615889, PMID:9692889 Sources: GOC:mgi_curators